{
  "term_label": "O-methyltransferase activity",
  "gene_symbol": "MEPCE",
  "gene_name": "7SK snRNA methylphosphate capping enzyme",
  "gene": "UniProtKB:Q7L2J0",
  "term_id": "GO:0008171"
}